negative regulation of NMDA glutamate receptor activity [GO:1904782] (biological process) Relationships: is a type of negative regulation of ion transmembrane transporter activity [GO:0032413]; is a type of negative regulation of signaling receptor activity [GO:2000272]; is_a regulation of NMDA receptor activity [GO:2000310]; negatively regulates NMDA glutamate receptor activity [GO:0004972] Definition: Any process that stops, prevents or reduces the frequency, rate or extent of NMDA glutamate receptor activity. References: PMID:12857 Sources: GOC:TermGenie, GOC:mr, GO_REF:0000059 Also known as: down regulation of N-methyl-D-aspartate selective glutamate receptor activity, down regulation of NMDA glutamate receptor activity, down regulation of NMDA receptor, down-regulation of N-methyl-D-aspartate selective glutamate receptor activity, down-regulation of NMDA glutamate receptor activity, down-regulation of NMDA receptor, downregulation of N-methyl-D-aspartate selective glutamate receptor activity, downregulation of NMDA glutamate receptor activity, downregulation of NMDA receptor, negative regulation of N-methyl-D-aspartate selective glutamate receptor activity, negative regulation of NMDA receptor, inhibition of N-methyl-D-aspartate selective glutamate receptor activity, inhibition of NMDA glutamate receptor activity, inhibition of NMDA receptor